positive regulation of blood circulation [GO:1903524] (biological process) Also known as: up regulation of blood circulation, up-regulation of blood circulation, upregulation of blood circulation, activation of blood circulation, activation of hemolymph circulation, positive regulation of hemolymph circulation, up regulation of hemolymph circulation, up-regulation of hemolymph circulation, upregulation of hemolymph circulation References: PMID:10659969 Sources: GOC:TermGenie, GOC:mr, GO_REF:0000058 Relationships: is a type of GO:0051240; is a type of regulation of blood circulation [GO:1903522]; positively regulates GO:0008015 Definition: Any process that activates or increases the frequency, rate or extent of blood circulation. Subtypes: positive regulation of heart contraction [GO:0045823], GO:0120277, positive regulation of gastric mucosal blood circulation [GO:1904346]